{
  "gene": "UniProtKB:Q9Y5N1",
  "term_id": "GO:0004969",
  "gene_name": "Histamine H3 receptor",
  "term_label": "histamine receptor activity",
  "gene_symbol": "HRH3"
}